{
  "gene_symbol": "CD33",
  "term_label": "plasma membrane",
  "term_id": "GO:0005886",
  "gene": "UniProtKB:P20138",
  "gene_name": "Myeloid cell surface antigen CD33"
}